{
  "gene": "UniProtKB:Q5VUD6",
  "gene_name": "Divergent protein kinase domain 1B",
  "term_label": "Unknown cellular component",
  "term_id": "UNKNOWN:0003",
  "gene_symbol": "DIPK1B"
}